{
  "gene": "UniProtKB:O60844",
  "gene_name": "Zymogen granule membrane protein 16",
  "gene_symbol": "ZG16",
  "term_label": "Unknown biological process",
  "term_id": "UNKNOWN:0002"
}